{
  "gene": "UniProtKB:Q96RD9",
  "gene_name": "Fc receptor-like protein 5",
  "gene_symbol": "FCRL5",
  "term_id": "GO:0006955",
  "term_label": "immune response"
}